{
  "gene_symbol": "RBFA",
  "gene": "UniProtKB:Q8N0V3",
  "gene_name": "Putative ribosome-binding factor A, mitochondrial",
  "term_label": "Unknown biological process",
  "term_id": "UNKNOWN:0002"
}